mannosyl-3-phosphoglycerate phosphatase activity [GO:0050531] (molecular function) Sources: EC:3.1.3.70, RHEA:19309 Relationships: is a type of phosphatase activity [GO:0016791] Definition: Catalysis of the reaction: 2-(alpha-D-mannosyl)-3-phosphoglycerate + H2O = 2-(alpha-D-mannosyl)-D-glycerate + phosphate. Also known as: alpha-D-mannosyl-3-phosphoglycerate phosphohydrolase activity